{
  "gene_symbol": "PHC2",
  "gene_name": "Polyhomeotic-like protein 2",
  "term_id": "GO:0003682",
  "term_label": "chromatin binding",
  "gene": "UniProtKB:Q8IXK0"
}